P-type calcium transporter activity involved in regulation of presynaptic cytosolic calcium ion concentration [GO:1905056] (molecular function) Definition: A calcium-transporting P-type ATPase activity involved in regulation of presynaptic cytosolic calcium ion concentration. Relationships: is a type of P-type calcium transporter activity [GO:0005388]; is part of regulation of presynaptic cytosolic calcium ion concentration [GO:0099509] Also known as: ATP phosphohydrolase (Ca2+-transporting) involved in regulation of presynaptic cytosolic calcium ion concentration, ATPase-coupled calcium ion transmembrane transporter activity involved in regulation of presynaptic cytosolic calcium levels, Ca(2+)-transporting ATPase activity involved in regulation of presynaptic cytosolic calcium ion concentration, Ca2+-pumping ATPase activity involved in regulation of presynaptic cytosolic calcium ion concentration, Ca2+-transporting ATPase activity involved in regulation of presynaptic cytosolic calcium ion concentration, calcium transporting ATPase activity involved in regulation of presynaptic cytosolic calcium ion concentration, calcium-transporting ATPase activity involved in regulation of presynaptic cytosolic calcium ion concentration, calcium ABC transporter involved in regulation of presynaptic cytosolic calcium ion concentration, calcium efflux ATPase involved in regulation of presynaptic cytosolic calcium ion concentration, calcium-translocating P-type ATPase activity involved in regulation of presynaptic cytosolic calcium ion concentration, plasma membrane Ca-ATPase involved in regulation of presynaptic cytosolic calcium ion concentration References: PMID:22972962 Sources: GOC:TermGenie, GO_REF:0000061